{
  "term_id": "GO:0030970",
  "gene_symbol": "SELENOS",
  "gene": "UniProtKB:Q9BQE4",
  "term_label": "retrograde protein transport, ER to cytosol",
  "gene_name": "Selenoprotein S"
}